{
  "term_id": "GO:0005634",
  "gene": "UniProtKB:Q16384",
  "term_label": "nucleus",
  "gene_symbol": "SSX1",
  "gene_name": "Protein SSX1"
}